{
  "term_id": "GO:0000137",
  "term_label": "Golgi cis cisterna",
  "gene": "UniProtKB:H3BV12",
  "gene_symbol": "GOLGA8Q",
  "gene_name": "Golgin subfamily A member 8Q"
}